{
  "term_id": "GO:0005886",
  "term_label": "plasma membrane",
  "gene_name": "Organic solute transporter subunit alpha",
  "gene_symbol": "SLC51A",
  "gene": "UniProtKB:Q86UW1"
}